{
  "term_id": "GO:0022857",
  "gene": "UniProtKB:Q8N4M1",
  "gene_name": "Choline transporter-like protein 3",
  "gene_symbol": "SLC44A3",
  "term_label": "transmembrane transporter activity"
}